regulation of secretion [GO:0051046] (BP) Definition: Any process that modulates the frequency, rate or extent of the controlled release of a substance from a cell or a tissue. Relationships: is a type of regulation of transport [GO:0051049]; regulates secretion [GO:0046903] Sources: GOC:ai Subtypes: regulation of peptide secretion [GO:0002791], regulation of gamma-aminobutyric acid secretion [GO:0014052], regulation of icosanoid secretion [GO:0032303], regulation of excretion [GO:0044062], regulation of saliva secretion [GO:0046877], GO:0051047, negative regulation of secretion [GO:0051048], regulation of gastric acid secretion [GO:0060453], GO:0070255, GO:0090165, regulation of pancreatic juice secretion [GO:0090186], regulation of bile acid secretion [GO:0120188], regulation of lactation [GO:1903487], regulation of secretion by cell [GO:1903530]